{
  "gene": "UniProtKB:A0A087X1G2",
  "term_id": "UNKNOWN:0002",
  "gene_name": "TBC1 domain family member 3K",
  "term_label": "Unknown biological process",
  "gene_symbol": "TBC1D3K"
}